spinal cord motor neuron differentiation [GO:0021522] (biological process) Definition: The process in which neuroepithelial cells in the ventral neural tube acquire specialized structural and/or functional features of motor neurons. Motor neurons innervate an effector (muscle or glandular) tissue and are responsible for transmission of motor impulses from the brain to the periphery. Differentiation includes the processes involved in commitment of a cell to a specific fate. Relationships: is_a cell differentiation in spinal cord [GO:0021515]; is a type of central nervous system neuron differentiation [GO:0021953]; is part of ventral spinal cord development [GO:0021517] References: PMID:11262869 Sources: GOC:cls, GOC:dgh, GOC:dph, GOC:jid, GO_REF:0000021 Subtypes: somatic motor neuron differentiation [GO:0021523], visceral motor neuron differentiation [GO:0021524], lateral motor column neuron differentiation [GO:0021525]